{
  "term_id": "UNKNOWN:0003",
  "gene_name": "Putative uncharacterized protein encoded by LINC00167",
  "term_label": "Unknown cellular component",
  "gene_symbol": "PRDM10-DT",
  "gene": "UniProtKB:Q96N53"
}